{
  "gene_name": "Annexin A7",
  "term_label": "plasma membrane",
  "gene_symbol": "ANXA7",
  "gene": "UniProtKB:P20073",
  "term_id": "GO:0005886"
}